{
  "term_label": "receptor ligand activity",
  "gene_symbol": "ULBP1",
  "term_id": "GO:0048018",
  "gene": "UniProtKB:Q9BZM6",
  "gene_name": "UL16-binding protein 1"
}